mRNA phosphatase activator activity [GO:0170008] (molecular function) Relationships: is a type of enzyme activator activity [GO:0008047]; positively regulates mRNA 5'-triphosphate monophosphatase activity [GO:0140818] Definition: Binds to and increases the activity of mRNA phosphatase. References: PMID:22323607